phenotypic switching [GO:0036166] (biological process) Subtypes: GO:0090677 Also known as: phenotypic dimorphism Definition: A reversible switch of a cell from one cell type or form to another, at a frequency above the expected frequency for somatic mutations. Phenotypic switching involves changes in cell morphology and altered gene expression patterns. For example, Candida albicans switches from white cells to opaque cells for sexual mating. Phenotypic switching also occurs in multicellular organisms; smooth muscle cells (SMCs) exhibit phenotypic transitions to allow rapid adaption to fluctuating environmental cues. Note: Mating type switching is not considered a type of phenotypic switching: for mating type switching, consider instead annotating to 'mating type switching ; GO:0007533'. Relationships: is a type of cellular process [GO:0009987] References: PMID:12443899, PMID:22406749, PMID:8456504 Sources: GOC:bf, GOC:di, Wikipedia:Phenotypic_switching Regulation: RO_0002211 by regulation of phenotypic switching [GO:1900239]; negatively regulated by negative regulation of phenotypic switching [GO:1900240]; positively regulated by positive regulation of phenotypic switching [GO:1900241]